{
  "term_id": "UNKNOWN:0002",
  "gene": "UniProtKB:Q6P2D8",
  "gene_name": "X-ray radiation resistance-associated protein 1",
  "gene_symbol": "XRRA1",
  "term_label": "Unknown biological process"
}